{
  "gene_name": "Putative uncharacterized protein UNQ5815_PRO19632",
  "gene": "UniProtKB:Q6UWF5",
  "term_id": "UNKNOWN:0001",
  "term_label": "Unknown molecular function",
  "gene_symbol": "UNQ5815_PRO19632"
}